{
  "gene_name": "ATP-binding cassette sub-family A member 2",
  "term_label": "Unknown cellular component",
  "gene": "UniProtKB:Q9BZC7",
  "gene_symbol": "ABCA2",
  "term_id": "UNKNOWN:0003"
}